{
  "term_label": "Unknown biological process",
  "gene": "UniProtKB:Q8N7R1",
  "term_id": "UNKNOWN:0002",
  "gene_symbol": "POM121L12",
  "gene_name": "POM121-like protein 12"
}